{
  "term_id": "UNKNOWN:0002",
  "gene": "UniProtKB:Q8N5W8",
  "term_label": "Unknown biological process",
  "gene_symbol": "FAM24B",
  "gene_name": "Protein FAM24B"
}